{
  "term_id": "GO:0003950",
  "gene_name": "Ecto-ADP-ribosyltransferase 3",
  "term_label": "NAD+ poly-ADP-ribosyltransferase activity",
  "gene_symbol": "ART3",
  "gene": "UniProtKB:Q13508"
}